embryo development ending in birth or egg hatching [GO:0009792] (biological process) Subtypes: embryonic development via the syncytial blastoderm [GO:0001700], GO:0043009 Also known as: embryogenesis Sources: GOC:go_curators, GOC:isa_complete, GOC:mtg_sensu Definition: The process whose specific outcome is the progression of an embryo over time, from zygote formation until the end of the embryonic life stage. The end of the embryonic life stage is organism-specific and may be somewhat arbitrary; for mammals it is usually considered to be birth, for insects the hatching of the first instar larva from the eggshell. Relationships: is a type of embryo development [GO:0009790]